{
  "gene_symbol": "NDUFS4",
  "gene_name": "NADH dehydrogenase [ubiquinone] iron-sulfur protein 4, mitochondrial",
  "term_label": "Unknown molecular function",
  "term_id": "UNKNOWN:0001",
  "gene": "UniProtKB:O43181"
}